ISGF3 complex [GO:0070721] (cellular component) Also known as: interferon-stimulated gene factor 3 transcription complex Relationships: is a type of RNA polymerase II transcription regulator complex [GO:0090575] Definition: A transcription factor complex that consists of a Stat1-Stat2 heterodimer and the IRF9 protein. References: PMID:8943351 Sources: GOC:mah